carbazole 1,9a-dioxygenase [NAD(P)H] activity [GO:0018564] (molecular function) Sources: EC:1.14.12.22 Relationships: is a type of oxidoreductase activity, acting on paired donors, with incorporation or reduction of molecular oxygen, NAD(P)H as one donor, and incorporation of two atoms of oxygen into one donor [GO:0016708] Definition: Catalysis of the reaction: 9H-carbazole + H+ + NAD(P)H + O2 = 2'-aminobiphenyl-2,3-diol + NAD(P)+. Also known as: CARDO, carbazole 1,9alpha-dioxygenase activity